{
  "term_id": "GO:0046923",
  "gene_symbol": "KDELR2",
  "gene_name": "ER lumen protein-retaining receptor 2",
  "term_label": "ER retention sequence binding",
  "gene": "UniProtKB:P33947"
}